{
  "gene_name": "Protein FAM210A",
  "term_id": "GO:0005739",
  "gene_symbol": "FAM210A",
  "term_label": "mitochondrion",
  "gene": "UniProtKB:Q96ND0"
}